{
  "gene_symbol": "BCAR3",
  "gene": "UniProtKB:O75815",
  "term_label": "insulin receptor signaling pathway",
  "term_id": "GO:0008286",
  "gene_name": "Breast cancer anti-estrogen resistance protein 3"
}